{
  "gene_symbol": "TUBGCP6",
  "gene_name": "Gamma-tubulin complex component 6",
  "term_id": "GO:0007020",
  "gene": "UniProtKB:Q96RT7",
  "term_label": "microtubule nucleation"
}